{
  "term_id": "GO:1905355",
  "term_label": "spine apparatus assembly",
  "gene_symbol": "SYNPO",
  "gene_name": "Synaptopodin",
  "gene": "UniProtKB:Q8N3V7"
}